{
  "gene_name": "Ubiquitin-conjugating enzyme E2 W",
  "term_label": "nucleus",
  "gene_symbol": "UBE2W",
  "gene": "UniProtKB:Q96B02",
  "term_id": "GO:0005634"
}